vitexin beta-glucosyltransferase activity [GO:0050395] (molecular function) Sources: EC:2.4.1.105, RHEA:21956 Also known as: vitexin b-glucosyltransferase activity, UDP-glucose:vitexin 2''-O-beta-D-glucosyltransferase activity, UDPglucose:vitexin 2''-O-beta-D-glucosyltransferase activity, uridine diphosphoglucose-vitexin 2''-glucosyltransferase activity Relationships: is a type of GO:0035251 Definition: Catalysis of the reaction: UDP-D-glucose + vitexin = H+ + UDP + vitexin 2''-O-beta-D-glucoside.